{
  "gene": "UniProtKB:O14618",
  "gene_symbol": "CCS",
  "term_label": "copper ion binding",
  "term_id": "GO:0005507",
  "gene_name": "Copper chaperone for superoxide dismutase"
}